{
  "term_id": "UNKNOWN:0001",
  "gene_symbol": "GTPBP8",
  "term_label": "Unknown molecular function",
  "gene_name": "GTP-binding protein 8",
  "gene": "UniProtKB:Q8N3Z3"
}